{
  "gene_symbol": "ZBTB40",
  "term_id": "GO:0006357",
  "term_label": "regulation of transcription by RNA polymerase II",
  "gene": "UniProtKB:Q9NUA8",
  "gene_name": "Zinc finger and BTB domain-containing protein 40"
}